cyclopropane-fatty-acyl-phospholipid synthase activity [GO:0008825] (MF) Definition: Catalysis of the reaction: S-adenosyl-L-methionine + phospholipid olefinic fatty acid = S-adenosyl-L-homocysteine + phospholipid cyclopropane fatty acid. Sources: EC:2.1.1.79 Also known as: cyclopropane synthetase activity, unsaturated-phospholipid methyltransferase activity, CFA synthase activity, S-adenosyl-L-methionine:unsaturated-phospholipid methyltransferase (cyclizing), cyclopropane fatty acid synthase activity, cyclopropane fatty acid synthetase activity, cyclopropane synthase activity Relationships: is a type of S-adenosylmethionine-dependent methyltransferase activity [GO:0008757]